slow endocytic recycling [GO:0032458] (biological process) References: PMID:16473635 Sources: GOC:ecd Definition: The directed movement of membrane-bounded vesicles from deep (non-peripheral) compartments endocytic compartments back to the plasma membrane where they are recycled for further rounds of transport. Relationships: is a type of endocytic recycling [GO:0032456]